{
  "gene_symbol": "NRXN3",
  "term_label": "gephyrin clustering involved in postsynaptic density assembly",
  "gene_name": "Neurexin-3",
  "gene": "UniProtKB:Q9Y4C0",
  "term_id": "GO:0097116"
}